{
  "gene_name": "Nicotinamide_nicotinic acid mononucleotide adenylyltransferase 3",
  "gene_symbol": "NMNAT3",
  "gene": "UniProtKB:Q96T66",
  "term_label": "nicotinamide-nucleotide adenylyltransferase activity",
  "term_id": "GO:0000309"
}